{
  "term_label": "DNA damage response",
  "gene": "UniProtKB:Q9NPI8",
  "gene_symbol": "FANCF",
  "gene_name": "Fanconi anemia group F protein",
  "term_id": "GO:0006974"
}